{
  "term_id": "UNKNOWN:0003",
  "term_label": "Unknown cellular component",
  "gene": "UniProtKB:Q8WUJ3",
  "gene_name": "Cell migration-inducing and hyaluronan-binding protein",
  "gene_symbol": "CEMIP"
}